{
  "gene_name": "Anoctamin-8",
  "gene_symbol": "ANO8",
  "gene": "UniProtKB:Q9HCE9",
  "term_label": "Unknown molecular function",
  "term_id": "UNKNOWN:0001"
}